{
  "gene_symbol": "PLOD1",
  "term_id": "GO:0005794",
  "gene_name": "Procollagen-lysine,2-oxoglutarate 5-dioxygenase 1",
  "gene": "UniProtKB:Q02809",
  "term_label": "Golgi apparatus"
}